vacuole inheritance [GO:0000011] (biological process) Relationships: is_a GO:0007033; is a type of GO:0048308 References: PMID:10873824, PMID:14616069 Sources: GOC:mcc Definition: The distribution of vacuoles into daughter cells after mitosis or meiosis, mediated by interactions between vacuoles and the cytoskeleton.